alpha1-beta1 integrin-tyrosine-protein phosphatase non-receptor type 2 complex [GO:0071124] (cellular component) Relationships: is a type of GO:0098797 References: PMID:15592458 Definition: A protein complex that consists of an alpha1-beta1 integrin complex bound to tyrosine-protein phosphatase non-receptor type 2. Also known as: ITGA1-ITGB1-PTPN2 complex